{
  "term_id": "GO:0046854",
  "gene_name": "Inositol hexakisphosphate kinase 1",
  "gene": "UniProtKB:Q92551",
  "gene_symbol": "IP6K1",
  "term_label": "phosphatidylinositol phosphate biosynthetic process"
}